{
  "gene": "UniProtKB:P35680",
  "term_id": "GO:0000978",
  "term_label": "RNA polymerase II cis-regulatory region sequence-specific DNA binding",
  "gene_name": "Hepatocyte nuclear factor 1-beta",
  "gene_symbol": "HNF1B"
}